{
  "gene_name": "Cytochrome c oxidase assembly protein COX18, mitochondrial",
  "term_id": "GO:0032977",
  "gene_symbol": "COX18",
  "gene": "UniProtKB:Q8N8Q8",
  "term_label": "membrane insertase activity"
}